{
  "gene": "UniProtKB:Q9NRR2",
  "gene_name": "Tryptase gamma",
  "gene_symbol": "TPSG1",
  "term_label": "proteolysis",
  "term_id": "GO:0006508"
}